{
  "gene_name": "Adhesion G-protein coupled receptor V1",
  "term_label": "stereocilium",
  "term_id": "GO:0032420",
  "gene_symbol": "ADGRV1",
  "gene": "UniProtKB:Q8WXG9"
}